spectrosome organization [GO:0030721] (biological process) References: PMID:11131529 Definition: A process that is carried out at the cellular level which results in the assembly, arrangement of constituent parts, or disassembly of the spectrosome, a germline specific spherical organelle that is the precursor to the fusome. Relationships: is a type of GO:0006996 Also known as: spectrosome organisation, spectrosome organization and biogenesis